{
  "term_label": "RNA catabolic process",
  "gene_name": "Ribonuclease H2 subunit B",
  "gene": "UniProtKB:Q5TBB1",
  "term_id": "GO:0006401",
  "gene_symbol": "RNASEH2B"
}